{
  "term_label": "Unknown cellular component",
  "term_id": "UNKNOWN:0003",
  "gene_name": "Transmembrane protein 106A",
  "gene": "UniProtKB:Q96A25",
  "gene_symbol": "TMEM106A"
}